rRNA (uridine-C5-)-methyltransferase activity [GO:0070041] (molecular function) Sources: GOC:imk, GOC:mah Relationships: is a type of GO:0008169; is a type of rRNA (uridine) methyltransferase activity [GO:0016436] Definition: Catalysis of the reaction: S-adenosyl-L-methionine + rRNA = S-adenosyl-L-homocysteine + rRNA containing C5-methyluridine.